{
  "gene": "UniProtKB:Q8NEB7",
  "gene_name": "Acrosin-binding protein",
  "gene_symbol": "ACRBP",
  "term_label": "acrosomal vesicle",
  "term_id": "GO:0001669"
}